metanephric tubule formation [GO:0072174] (biological process) Definition: The developmental process pertaining to the initial formation of a metanephric tubule. Subtypes: metanephric nephron tubule formation [GO:0072289] Relationships: is a type of GO:0072175; is part of metanephric tubule morphogenesis [GO:0072173] Sources: GOC:mtg_kidney_jan10